{
  "term_id": "UNKNOWN:0002",
  "gene_symbol": "ACTL9",
  "gene": "UniProtKB:Q8TC94",
  "gene_name": "Actin-like protein 9",
  "term_label": "Unknown biological process"
}